steroid hormone binding [GO:1990239] (molecular function) Definition: Binding to a steroid hormone. Relationships: is a type of steroid binding [GO:0005496]; is a type of hormone binding [GO:0042562] Sources: GOC:ln Subtypes: (25S)-Delta(4)-dafachronate binding [GO:1902051], (25S)-Delta(7)-dafachronate binding [GO:1902052], GO:1903794, GO:1903875, 11-deoxycortisol binding [GO:1903876], GO:1903878